{
  "gene_name": "Protein amnionless",
  "term_label": "apical plasma membrane",
  "gene": "UniProtKB:Q9BXJ7",
  "gene_symbol": "AMN",
  "term_id": "GO:0016324"
}